{
  "gene_symbol": "SAMD15",
  "gene": "UniProtKB:Q9P1V8",
  "gene_name": "Sterile alpha motif domain-containing protein 15",
  "term_label": "Unknown cellular component",
  "term_id": "UNKNOWN:0003"
}